detection of virus [GO:0009597] (biological process) Note: GO:0009597 is not a child term of 'detection of symbiont ; GO:0009602' to allow annotation of a virus responding to another (often competing) virus. Also known as: perception of virus Definition: The series of events in which a stimulus from a virus is received and converted into a molecular signal. Relationships: is a type of GO:0009615 Sources: GOC:hb